{
  "gene_symbol": "ZNF445",
  "gene_name": "Zinc finger protein 445",
  "term_id": "GO:0044726",
  "gene": "UniProtKB:P59923",
  "term_label": "epigenetic programing of female pronucleus"
}